{
  "term_label": "Unknown cellular component",
  "gene": "UniProtKB:Q6UXZ4",
  "gene_name": "Netrin receptor UNC5D",
  "term_id": "UNKNOWN:0003",
  "gene_symbol": "UNC5D"
}